cell differentiation involved in embryonic placenta development [GO:0060706] (biological process) Subtypes: epithelial cell differentiation involved in embryonic placenta development [GO:0060671], trophoblast giant cell differentiation [GO:0060707], GO:0060708, GO:0060709, GO:0060715 Sources: GOC:dph Regulation: regulated by regulation of cell differentiation involved in embryonic placenta development [GO:0060800]; negatively regulated by negative regulation of cell differentiation involved in embryonic placenta development [GO:0060806] Relationships: is a type of developmental process involved in reproduction [GO:0003006]; is a type of cell differentiation [GO:0030154]; is part of embryonic placenta development [GO:0001892] Definition: The process in which a relatively unspecialized cell acquires specialized features of the embryonic placenta.